{
  "gene_symbol": "CTAGE1",
  "term_label": "endoplasmic reticulum membrane",
  "gene_name": "cTAGE family member 2",
  "term_id": "GO:0005789",
  "gene": "UniProtKB:Q96RT6"
}